positive regulation of syringal lignin catabolic process [GO:1901471] (biological process) Definition: Any process that activates or increases the frequency, rate or extent of syringal lignin catabolic process. Also known as: activation of S-lignin catabolic process, activation of syringal lignin breakdown, activation of syringal lignin catabolism, activation of syringal lignin degradation, positive regulation of S-lignin catabolic process, positive regulation of syringal lignin breakdown, positive regulation of syringal lignin catabolism, positive regulation of syringal lignin degradation, up regulation of S-lignin catabolic process, up regulation of syringal lignin breakdown, up regulation of syringal lignin catabolic process, up regulation of syringal lignin catabolism, up regulation of syringal lignin degradation, up-regulation of S-lignin catabolic process, up-regulation of syringal lignin breakdown, up-regulation of syringal lignin catabolic process, up-regulation of syringal lignin catabolism, up-regulation of syringal lignin degradation, upregulation of S-lignin catabolic process, upregulation of syringal lignin breakdown, upregulation of syringal lignin catabolic process, upregulation of syringal lignin catabolism, upregulation of syringal lignin degradation, activation of syringal lignin catabolic process Sources: GOC:TermGenie, GOC:mengo_curators Relationships: is a type of positive regulation of catabolic process [GO:0009896]; is a type of regulation of syringal lignin catabolic process [GO:1901469]; positively regulates syringal lignin catabolic process [GO:1901065]